{
  "term_id": "GO:0000727",
  "term_label": "double-strand break repair via break-induced replication",
  "gene": "UniProtKB:P33993",
  "gene_symbol": "MCM7",
  "gene_name": "DNA replication licensing factor MCM7"
}